{
  "term_id": "GO:0007005",
  "gene_name": "Coiled-coil-helix-coiled-coil-helix domain-containing protein 2",
  "gene_symbol": "CHCHD2",
  "term_label": "mitochondrion organization",
  "gene": "UniProtKB:Q9Y6H1"
}